{
  "gene_symbol": "TTLL5",
  "gene_name": "Tubulin polyglutamylase TTLL5",
  "gene": "UniProtKB:Q6EMB2",
  "term_label": "ciliary basal body",
  "term_id": "GO:0036064"
}